{
  "gene_symbol": "DRAXIN",
  "gene": "UniProtKB:Q8NBI3",
  "term_id": "GO:0007411",
  "term_label": "axon guidance",
  "gene_name": "Draxin"
}